{
  "term_id": "GO:0031071",
  "gene_symbol": "NFS1",
  "gene_name": "Cysteine desulfurase",
  "term_label": "cysteine desulfurase activity",
  "gene": "UniProtKB:Q9Y697"
}